natural killer cell cytokine production [GO:0002370] (biological process) Relationships: is a type of natural killer cell mediated immunity [GO:0002228]; is a type of cytokine production involved in immune response [GO:0002367] Regulation: regulated by GO:0002727; negatively regulated by negative regulation of natural killer cell cytokine production [GO:0002728]; positively regulated by positive regulation of natural killer cell cytokine production [GO:0002729] Definition: Any process that contributes to cytokine production by a natural killer cell. Note: Note that this term is in the subset of terms that should not be used for direct gene product annotation. Instead, select one of the 'regulation' children terms. Also known as: NK cell cytokine production Sources: GOC:add, ISBN:0781735149